{
  "gene_symbol": "LCN1",
  "gene_name": "Lipocalin-1",
  "term_label": "Unknown biological process",
  "gene": "UniProtKB:P31025",
  "term_id": "UNKNOWN:0002"
}